styrene catabolic process [GO:0042207] (biological process) Sources: GOC:jl Relationships: is a type of GO:0018966; is a type of xenobiotic catabolic process [GO:0042178]; is a type of hydrocarbon catabolic process [GO:0120253]; is a type of GO:0120256 Definition: The chemical reactions and pathways resulting in the breakdown of styrene, an aromatic hydrocarbon liquid used in the manufacture of polystyrene. Also known as: styrene breakdown, styrene catabolism, styrene degradation